{
  "term_id": "GO:0015035",
  "gene": "UniProtKB:Q9NS18",
  "term_label": "protein-disulfide reductase activity",
  "gene_name": "Glutaredoxin-2, mitochondrial",
  "gene_symbol": "GLRX2"
}